{
  "gene": "UniProtKB:Q9BZM5",
  "gene_symbol": "ULBP2",
  "gene_name": "UL16-binding protein 2",
  "term_label": "receptor ligand activity",
  "term_id": "GO:0048018"
}